{
  "gene_name": "Cadherin-4",
  "gene": "UniProtKB:P55283",
  "term_id": "GO:0016477",
  "term_label": "cell migration",
  "gene_symbol": "CDH4"
}